regulation of fusion of virus membrane with host plasma membrane [GO:1903913] (biological process) Subtypes: negative regulation of fusion of virus membrane with host plasma membrane [GO:1903914], positive regulation of fusion of virus membrane with host plasma membrane [GO:1903915] Also known as: regulation of viral envelope fusion, regulation of viral envelope fusion with host cell membrane, regulation of viral envelope fusion with host membrane, regulation of viral envelope fusion with host plasma membrane, regulation of viral penetration via membrane fusion, regulation of viral entry into host cell via membrane fusion with the plasma membrane, regulation of viral-cell fusion molecule activity Relationships: is a type of regulation of viral entry into host cell [GO:0046596]; is a type of regulation of cellular component organization [GO:0051128]; regulates fusion of virus membrane with host plasma membrane [GO:0019064] References: PMID:23575248 Sources: GOC:TermGenie, GOC:als, GO_REF:0000058 Definition: Any process that modulates the frequency, rate or extent of fusion of virus membrane with host plasma membrane.